{
  "term_label": "dipeptidyl-peptidase activity",
  "gene": "UniProtKB:Q12884",
  "gene_name": "Prolyl endopeptidase FAP",
  "gene_symbol": "FAP",
  "term_id": "GO:0008239"
}